flavonol-3-O-glycoside xylosyltransferase activity [GO:0047285] (molecular function) Definition: Catalysis of the reaction: flavonol 3-O-glycoside + UDP-D-xylose = flavonol 3-O-D-xylosylglycoside + UDP. Also known as: UDP-D-xylose:flavonol-3-O-glycoside 2''-O-beta-D-xylosyltransferase activity Relationships: is a type of UDP-xylosyltransferase activity [GO:0035252] Sources: EC:2.4.2.35, MetaCyc:2.4.2.35-RXN